venom-mediated perturbation of muscle system process [GO:0140137] (biological process) Sources: GOC:pg Definition: A process in which an organism alters or subverts a muscular process in another organism via the action of a venom. Subtypes: venom-mediated smooth muscle relaxation [GO:0044617] Relationships: is a type of GO:0035738